{
  "term_label": "Unknown molecular function",
  "gene_symbol": "CDCA7L",
  "term_id": "UNKNOWN:0001",
  "gene": "UniProtKB:Q96GN5",
  "gene_name": "Cell division cycle-associated 7-like protein"
}